{
  "gene_name": "NALCN channel auxiliary factor 2",
  "term_id": "GO:0098703",
  "gene_symbol": "NALF2",
  "term_label": "calcium ion import across plasma membrane",
  "gene": "UniProtKB:O75949"
}